response to nitrogen compound [GO:1901698] (BP) Also known as: response to nitrogen molecular entity Relationships: is a type of GO:0042221 Definition: Any process that results in a change in state or activity of a cell or an organism (in terms of movement, secretion, enzyme production, gene expression, etc.) as a result of a nitrogen compound stimulus. Subtypes: response to 1-aminocyclopropane-1-carboxylic acid [GO:0009961], response to nitrate [GO:0010167], GO:0010200, response to proline [GO:0010238], response to vitamin B1 [GO:0010266], response to purine-containing compound [GO:0014074], response to amine [GO:0014075], response to methotrexate [GO:0031427], mRNA export from nucleus in response to heat stress [GO:0031990], GO:0032494, GO:0032495, response to vitamin B2 [GO:0033274], GO:0033590, response to vitamin B6 [GO:0034516], response to histamine [GO:0034776], GO:0035713, response to trichostatin A [GO:0035983], GO:0036272, response to lapatinib [GO:0036274], response to ximelagatran [GO:0036288], ERAD pathway [GO:0036503], GO:0043201, response to alkaloid [GO:0043279], response to dsRNA [GO:0043331], response to peptide hormone [GO:0043434], response to bacteriocin [GO:0046678], GO:0046681, response to cycloheximide [GO:0046898], response to folic acid [GO:0051593], response to lipoprotein particle [GO:0055094], response to ammonium ion [GO:0060359], response to (R)-carnitine [GO:0061959], response to biotin [GO:0070781], response to heparin [GO:0071503], response to indole-3-methanol [GO:0071680], response to nitric oxide [GO:0071731], response to monoamine [GO:0071867], GO:0072710, response to thiabendazole [GO:0072712], response to actinomycin D [GO:0072716], response to amitrole [GO:0072722], GO:0072724, response to diamide [GO:0072737], response to indolebutyric acid [GO:0080026], GO:0080033, response to histidine [GO:0080052], GO:0080053, response to azide [GO:0097184], response to 5-fluoro-2'-deoxyuridine [GO:0097330], response to cytarabine [GO:0097331], response to olanzapine [GO:0097333], response to perphenazine [GO:0097334], response to quetiapine [GO:0097335], response to risperidone [GO:0097336], response to ziprasidone [GO:0097337], response to clozapine [GO:0097338], stress-induced homeostatically regulated protein degradation pathway [GO:0120174], response to chloramphenicol [GO:1901322], response to antimycin A [GO:1901325], response to tacrolimus [GO:1901327], response to cytochalasin B [GO:1901328], response to L-thialysine [GO:1901345], response to L-canavanine [GO:1901354], response to rapamycin [GO:1901355], response to L-cysteine [GO:1901367], response to glutathione [GO:1901370], GO:1901554, response to candesartan [GO:1901556], response to metformin [GO:1901558], response to ribavirin [GO:1901559], response to GW 7647 [GO:1901593], response to capsazepine [GO:1901594], response to carbendazim [GO:1901597], cellular response to nitrogen compound [GO:1901699], response to ketamine [GO:1901986], response to L-glutamate [GO:1902065], response to chloroquine [GO:1902349], response to imidacloprid [GO:1902351], response to cyclophosphamide [GO:1902518], response to doxorubicin [GO:1902520], response to 4'-epidoxorubicin [GO:1902522], response to clopidogrel [GO:1903493], response to L-arginine [GO:1903576], response to acrylamide [GO:1903937], response to micafungin [GO:1903967], response to acadesine [GO:1904101], response to desipramine [GO:1904307], response to 2-O-acetyl-1-O-hexadecyl-sn-glycero-3-phosphocholine [GO:1904316], GO:1904373, response to L-phenylalanine derivative [GO:1904386], response to ciliary neurotrophic factor [GO:1904391], response to nocodazole [GO:1904402], response to tetrahydrofolate [GO:1904481], GO:1904560, response to polyamine macromolecule [GO:1904583], GO:1904585, response to glycoprotein [GO:1904587], response to methionine [GO:1904640], response to dinitrophenol [GO:1904641], response to amyloid-beta [GO:1904645], response to nitroglycerin [GO:1904842], response to L-glutamine [GO:1904844], response to bleomycin [GO:1904975], GO:1905119, response to acetylcholine [GO:1905144], response to cyclosporin A [GO:1905237], response to 3,3',5-triiodo-L-thyronine [GO:1905242], response to miconazole [GO:1905307], response to homocysteine [GO:1905374], GO:1905429, response to chondroitin 6'-sulfate [GO:1905439], response to chondroitin 4'-sulfate [GO:1905441], response to pyrimidine ribonucleotide [GO:1905834], response to temozolomide [GO:1990054], response to dsDNA [GO:1990784] Sources: GOC:TermGenie, GOC:pr Note: Note that this term is in the subset of terms that should not be used for direct gene product annotation. Instead, select a child term or, if no appropriate child term exists, please request a new term. Direct annotations to this term may be amended during annotation QC.